{
  "gene": "UniProtKB:Q5FWF5",
  "term_id": "GO:0000785",
  "gene_name": "N-acetyltransferase ESCO1",
  "term_label": "chromatin",
  "gene_symbol": "ESCO1"
}